{
  "term_label": "regulation of transcription by RNA polymerase II",
  "gene": "UniProtKB:Q08AN1",
  "gene_symbol": "ZNF616",
  "term_id": "GO:0006357",
  "gene_name": "Zinc finger protein 616"
}